flavonoid phytoalexin biosynthetic process [GO:0009716] (biological process) Sources: ISBN:0198506732 Also known as: flavonoid phytoalexin anabolism, flavonoid phytoalexin biosynthesis, flavonoid phytoalexin formation, flavonoid phytoalexin synthesis Relationships: is_a GO:0009813; is_a GO:0052315 Definition: The chemical reactions and pathways resulting in the formation of flavonoid phytoalexins, a group of water-soluble phenolic derivatives containing a flavan skeleton, which possess antibiotic activity and are produced by plant tissues in response to infection.